{
  "gene_name": "Forkhead box protein O3",
  "gene": "UniProtKB:O43524",
  "term_label": "DNA-binding transcription factor activity, RNA polymerase II-specific",
  "term_id": "GO:0000981",
  "gene_symbol": "FOXO3"
}